alcohol-forming long-chain fatty acyl-CoA reductase activity [GO:0102965] (molecular function) Relationships: is a type of oxidoreductase activity, acting on the aldehyde or oxo group of donors, NAD or NADP as acceptor [GO:0016620] Definition: Catalysis of the reaction: a long-chain fatty acyl-CoA + 2 H+ + 2 NADPH = a long-chain primary fatty alcohol + CoA + 2 NADP+. A long-chain fatty acid has an aliphatic tail containing 13 to 22 carbons. Sources: GOC:pz, RHEA:52716 Note: While there is not universal consensus on the lengths of short-, medium-, long- and very-long-chain fatty acids, the GO uses the definitions in ChEBI (see CHEBI:26666, CHEBI:59554, CHEBI:15904 and CHEBI:27283). Also known as: alcohol-forming fatty acyl-CoA reductase activity